positive regulation of anion transmembrane transport [GO:1903961] (biological process) Definition: Any process that activates or increases the frequency, rate or extent of anion transmembrane transport. Relationships: is a type of positive regulation of monoatomic ion transmembrane transport [GO:0034767]; is a type of positive regulation of monoatomic anion transport [GO:1903793]; is a type of regulation of monoatomic anion transmembrane transport [GO:1903959]; positively regulates monoatomic anion transmembrane transport [GO:0098656] Also known as: up regulation of anion transmembrane transport, up-regulation of anion transmembrane transport, upregulation of anion transmembrane transport, activation of anion transmembrane transport Sources: GOC:TermGenie, GOC:vw, GO_REF:0000058 Subtypes: positive regulation of anion channel activity [GO:1901529], GO:1904214